{
  "term_label": "endoplasmic reticulum membrane",
  "term_id": "GO:0005789",
  "gene": "UniProtKB:Q92903",
  "gene_name": "Phosphatidate cytidylyltransferase 1",
  "gene_symbol": "CDS1"
}